{
  "term_label": "brush border membrane",
  "term_id": "GO:0031526",
  "gene_name": "Guanine nucleotide-binding protein subunit alpha-13",
  "gene": "UniProtKB:Q14344",
  "gene_symbol": "GNA13"
}